butanal dehydrogenase [NAD(P)+] activity [GO:0047759] (molecular function) Definition: Catalysis of the reaction: butanal + CoA + NAD(P)+ = butanoyl-CoA + NAD(P)H + H+. Sources: EC:1.2.1.57, MetaCyc:BUTANAL-DEHYDROGENASE-RXN Relationships: is a type of aldehyde dehydrogenase [NAD(P)+] activity [GO:0004030] Also known as: butanal dehydrogenase activity, butanal:NAD(P)+ oxidoreductase (CoA-acylating)